{
  "gene_symbol": "PRO2829",
  "gene": "UniProtKB:Q9P1C3",
  "term_id": "UNKNOWN:0003",
  "term_label": "Unknown cellular component",
  "gene_name": "Putative uncharacterized protein PRO2829"
}